phenylethanolamine N-methyltransferase activity [GO:0004603] (molecular function) Also known as: S-adenosyl-L-methionine:phenylethanolamine N-methyltransferase activity, noradrenalin N-methyltransferase activity, noradrenaline N-methyltransferase activity, norepinephrine N-methyltransferase activity, norepinephrine methyltransferase activity, phenethanolamine N-methyltransferase activity, phenethanolamine methyltransferase activity Sources: EC:2.1.1.28 Definition: Catalysis of the reaction: S-adenosyl-L-methionine + phenylethanolamine = S-adenosyl-L-homocysteine + N-methylphenylethanolamine. Relationships: is a type of N-methyltransferase activity [GO:0008170]; is a type of S-adenosylmethionine-dependent methyltransferase activity [GO:0008757]